artery morphogenesis [GO:0048844] (biological process) Regulation: regulated by regulation of artery morphogenesis [GO:1905651]; negatively regulated by negative regulation of artery morphogenesis [GO:1905652]; positively regulated by positive regulation of artery morphogenesis [GO:1905653] Definition: The process in which the anatomical structures of arterial blood vessels are generated and organized. Arteries are blood vessels that transport blood from the heart to the body and its organs. Subtypes: aorta morphogenesis [GO:0035909], GO:0060982, pulmonary artery morphogenesis [GO:0061156], GO:0061441, pharyngeal arch artery morphogenesis [GO:0061626], ductus arteriosus closure [GO:0097070] Also known as: arterial morphogenesis, arteriogenesis References: PMID:16740480 Sources: GOC:dsf Relationships: is a type of blood vessel morphogenesis [GO:0048514]; is part of GO:0060840